{
  "term_label": "Unknown cellular component",
  "gene": "UniProtKB:A0N4Z8",
  "term_id": "UNKNOWN:0003",
  "gene_name": "HCG2039779 (Fragment)",
  "gene_symbol": "TRAJ9"
}